{
  "gene": "UniProtKB:P08319",
  "gene_symbol": "ADH4",
  "gene_name": "All-trans-retinol dehydrogenase [NAD(+)] ADH4",
  "term_id": "GO:0046294",
  "term_label": "formaldehyde catabolic process"
}